organellar chromatophore intermembrane space [GO:0070115] (cellular component) Sources: GOC:mah Also known as: Paulinella-type chromatophore intermembrane space Definition: The region between the inner and outer lipid bilayers that surround an organellar chromatophore. Relationships: is a type of cellular anatomical structure [GO:0110165]; is part of organellar chromatophore [GO:0070111]